{
  "gene_symbol": "IL27RA",
  "gene_name": "Interleukin-27 receptor subunit alpha",
  "term_label": "negative regulation of type 2 immune response",
  "term_id": "GO:0002829",
  "gene": "UniProtKB:Q6UWB1"
}